{
  "gene_name": "Norrin",
  "term_label": "Norrin signaling pathway",
  "gene": "UniProtKB:Q00604",
  "term_id": "GO:0110135",
  "gene_symbol": "NDP"
}